{
  "term_id": "UNKNOWN:0003",
  "gene": "UniProtKB:O43583",
  "gene_symbol": "DENR",
  "gene_name": "Density-regulated protein",
  "term_label": "Unknown cellular component"
}